{
  "term_label": "extracellular space",
  "gene": "UniProtKB:Q4G0M1",
  "gene_symbol": "ERFE",
  "term_id": "GO:0005615",
  "gene_name": "Erythroferrone"
}